{
  "gene_symbol": "MAP7",
  "gene_name": "Ensconsin",
  "term_id": "GO:0000226",
  "term_label": "microtubule cytoskeleton organization",
  "gene": "UniProtKB:Q14244"
}